{
  "gene_name": "pre-rRNA 2'-O-ribose RNA methyltransferase FTSJ3",
  "gene": "UniProtKB:Q8IY81",
  "gene_symbol": "FTSJ3",
  "term_label": "rRNA methylation",
  "term_id": "GO:0031167"
}